basal protein localization [GO:0045175] (biological process) Also known as: basal protein localisation, establishment and maintenance of basal protein localization, establishment and maintenance of protein localization in basal part of cell Definition: Any process in which a protein is transported to, or maintained in, basal regions of the cell. Relationships: is_a GO:0008104 Sources: GOC:bf